{
  "term_id": "GO:0003690",
  "gene_symbol": "PYHIN1",
  "term_label": "double-stranded DNA binding",
  "gene_name": "Pyrin and HIN domain-containing protein 1",
  "gene": "UniProtKB:Q6K0P9"
}